{
  "gene_name": "Putative dispanin subfamily A member 2d",
  "gene": "UniProtKB:C9JQL5",
  "gene_symbol": "C9JQL5",
  "term_id": "GO:0046597",
  "term_label": "host-mediated suppression of symbiont invasion"
}